{
  "term_label": "fructose 1,6-bisphosphate 1-phosphatase activity",
  "gene": "UniProtKB:P09467",
  "gene_symbol": "FBP1",
  "gene_name": "Fructose-1,6-bisphosphatase 1",
  "term_id": "GO:0042132"
}